L-cysteine desulfurase complex [GO:1990221] (cellular component) References: PMID:11827487 Sources: GOC:bhm Relationships: is a type of sulfurtransferase complex [GO:1990228] Definition: A protein complex capable of cysteine desulfurase activity decomposing L-cysteine to L-alanine and sulfur. It belongs to a ubiquitous family of pyridoxal 5-phosphate (PLP)-dependent enzymes. Also known as: IscS, NifS, SufS complex Subtypes: mitochondrial [2Fe-2S] assembly complex [GO:0099128], GO:1990329, IscS-IscU complex [GO:1990330]